{
  "gene": "UniProtKB:Q969P6",
  "term_id": "GO:0006260",
  "gene_symbol": "TOP1MT",
  "gene_name": "DNA topoisomerase I, mitochondrial",
  "term_label": "DNA replication"
}